positive regulation of dendritic cell differentiation [GO:2001200] (biological process) Definition: Any process that activates or increases the frequency, rate or extent of dendritic cell differentiation. Relationships: is a type of positive regulation of leukocyte differentiation [GO:1902107]; is a type of regulation of dendritic cell differentiation [GO:2001198]; positively regulates dendritic cell differentiation [GO:0097028] Sources: GOC:obol